chromosome, centromeric region [GO:0000775] (cellular component) Definition: The region of a chromosome that includes the centromeric DNA and associated proteins. In monocentric chromosomes, this region corresponds to a single area of the chromosome, whereas in holocentric chromosomes, it is evenly distributed along the chromosome. Note: Note that this term can be used in place of the obsolete cellular component term 'centromere ; GO:0005698'. Also known as: centromere complex, chromosome, centric region, centromere, chromosome, pericentric region Sources: GOC:cjm, GOC:elh, GOC:kmv, GOC:pr Relationships: is a type of chromosomal region [GO:0098687] Subtypes: condensed chromosome, centromeric region [GO:0000779]